{
  "gene_name": "Mpv17-like protein",
  "gene": "UniProtKB:Q2QL34",
  "term_label": "mitochondrion",
  "term_id": "GO:0005739",
  "gene_symbol": "MPV17L"
}